intermediate voltage-gated calcium channel activity [GO:1990028] (MF) References: PMID:16382099 Sources: GOC:BHF, GOC:rl, Wikipedia:Calcium_channel Also known as: R-type calcium channel Relationships: is a type of voltage-gated calcium channel activity [GO:0005245] Definition: Enables the transmembrane transfer of a calcium ion by an intermediate voltage-gated channel. An intermediate voltage-gated channel is a channel whose open state is dependent on intermediate voltage across the membrane in which it is embedded.